stress response to copper ion [GO:1990169] (biological process) Relationships: is_a GO:0046688; is_a stress response to metal ion [GO:0097501] Definition: Any process that results in a change in state or activity of a cell or an organism (in terms of movement, secretion, enzyme production, gene expression, etc.) as a result of a disturbance in organismal or cellular homeostasis caused by a copper ion stimulus. References: PMID:23437011 Sources: GOC:kmv Regulation: regulated by regulation of stress response to copper ion [GO:1903853]; RO_0002212 by negative regulation of stress response to copper ion [GO:1903854]; positively regulated by GO:1903855 Also known as: stress response to copper, response to copper ion stress, response to copper toxicity